{
  "gene": "UniProtKB:P10276",
  "gene_name": "Retinoic acid receptor alpha",
  "gene_symbol": "RARA",
  "term_id": "GO:0005634",
  "term_label": "nucleus"
}